{
  "gene_name": "Fibrous sheath-interacting protein 1",
  "gene_symbol": "FSIP1",
  "term_label": "Unknown molecular function",
  "gene": "UniProtKB:Q8NA03",
  "term_id": "UNKNOWN:0001"
}